{
  "term_label": "endoplasmic reticulum",
  "gene_name": "GPI inositol-deacylase",
  "term_id": "GO:0005783",
  "gene": "UniProtKB:Q75T13",
  "gene_symbol": "PGAP1"
}